{
  "term_label": "Unknown cellular component",
  "gene": "UniProtKB:Q6ZUT4",
  "gene_name": "Putative uncharacterized protein FLJ43343",
  "term_id": "UNKNOWN:0003",
  "gene_symbol": "Q6ZUT4"
}